{
  "term_id": "GO:1903561",
  "gene_symbol": "APOA5",
  "gene_name": "Apolipoprotein A-V",
  "term_label": "extracellular vesicle",
  "gene": "UniProtKB:Q6Q788"
}